glycerol kinase activity [GO:0004370] (molecular function) Relationships: is a type of kinase activity [GO:0016301]; is a type of GO:0016773 Definition: Catalysis of the reaction: ATP + glycerol = sn-glycerol 3-phosphate + ADP + 2 H+. Sources: EC:2.7.1.30, RHEA:21644 Also known as: ATP:glycerol 3-phosphotransferase activity, ATP:glycerol-3-phosphotransferase activity, GK, glyceric kinase activity, glycerokinase activity, glycerol kinase (phosphorylating)